{
  "gene_name": "Putative uncharacterized protein IGF2BP2-AS1",
  "term_label": "Unknown cellular component",
  "term_id": "UNKNOWN:0003",
  "gene_symbol": "IGF2BP2-AS1",
  "gene": "UniProtKB:Q96M15"
}